{
  "term_label": "GTPase activity",
  "gene": "UniProtKB:P29992",
  "gene_name": "Guanine nucleotide-binding protein subunit alpha-11",
  "gene_symbol": "GNA11",
  "term_id": "GO:0003924"
}